cellular response to radiation [GO:0071478] (biological process) Sources: GOC:mah Note: Note that 'radiation' refers to electromagnetic radiation of any wavelength. Also known as: cellular response to electromagnetic radiation stimulus, cellular response to radiation stimulus Relationships: is a type of response to radiation [GO:0009314]; is_a cellular response to abiotic stimulus [GO:0071214] Definition: Any process that results in a change in state or activity of a cell (in terms of movement, secretion, enzyme production, gene expression, etc.) as a result of an electromagnetic radiation stimulus. Electromagnetic radiation is a propagating wave in space with electric and magnetic components. These components oscillate at right angles to each other and to the direction of propagation. Subtypes: cellular response to ionizing radiation [GO:0071479], cellular response to light stimulus [GO:0071482]